{
  "term_label": "extracellular space",
  "gene_name": "Cystatin-C",
  "term_id": "GO:0005615",
  "gene_symbol": "CST3",
  "gene": "UniProtKB:P01034"
}